{
  "term_id": "GO:0000981",
  "gene": "UniProtKB:P43699",
  "gene_symbol": "NKX2-1",
  "term_label": "DNA-binding transcription factor activity, RNA polymerase II-specific",
  "gene_name": "Homeobox protein Nkx-2.1"
}